regulation of filamentous growth [GO:0010570] (biological process) Subtypes: negative regulation of filamentous growth [GO:0060258], GO:0090033, regulation of filamentous growth of a population of unicellular organisms [GO:1900428] Definition: Any process that modulates the frequency, rate or extent of the process in which a multicellular organism or a group of unicellular organisms grow in a threadlike, filamentous shape. Sources: GOC:dph, GOC:jp, GOC:tb Relationships: is a type of regulation of growth [GO:0040008]; RO_0002211 filamentous growth [GO:0030447]